{
  "term_id": "GO:0051306",
  "gene_symbol": "TEX14",
  "gene": "UniProtKB:Q8IWB6",
  "term_label": "mitotic sister chromatid separation",
  "gene_name": "Inactive serine_threonine-protein kinase TEX14"
}